{
  "term_label": "plasma membrane",
  "term_id": "GO:0005886",
  "gene": "UniProtKB:P30542",
  "gene_name": "Adenosine receptor A1",
  "gene_symbol": "ADORA1"
}